methyl-branched fatty acid biosynthetic process [GO:1902321] (biological process) Definition: The chemical reactions and pathways resulting in the formation of methyl-branched fatty acid. Relationships: is a type of fatty acid biosynthetic process [GO:0006633]; is a type of methyl-branched fatty acid metabolic process [GO:0097089] Regulation: regulated by GO:1902322; negatively regulated by negative regulation of methyl-branched fatty acid biosynthetic process [GO:1902323]; positively regulated by GO:1902324 References: PMID:15340492 Sources: GOC:TermGenie, GOC:kmv Also known as: methyl-branched fatty acid anabolism, methyl-branched fatty acid biosynthesis, methyl-branched fatty acid formation, methyl-branched fatty acid synthesis